{
  "term_label": "Unknown biological process",
  "gene": "UniProtKB:Q4G0G5",
  "gene_symbol": "SCGB2B2",
  "term_id": "UNKNOWN:0002",
  "gene_name": "Secretoglobin family 2B member 2"
}